{
  "gene_symbol": "VCP",
  "term_id": "GO:0030970",
  "gene": "UniProtKB:P55072",
  "gene_name": "Transitional endoplasmic reticulum ATPase",
  "term_label": "retrograde protein transport, ER to cytosol"
}